{
  "gene": "UniProtKB:Q96GD4",
  "gene_name": "Aurora kinase B",
  "gene_symbol": "AURKB",
  "term_id": "UNKNOWN:0001",
  "term_label": "Unknown molecular function"
}